{
  "term_label": "protein tyrosine phosphatase activity",
  "gene_symbol": "PTPRZ1",
  "gene": "UniProtKB:P23471",
  "term_id": "GO:0004725",
  "gene_name": "Receptor-type tyrosine-protein phosphatase zeta"
}